{
  "term_id": "UNKNOWN:0002",
  "gene": "UniProtKB:Q9UQ35",
  "term_label": "Unknown biological process",
  "gene_name": "Serine_arginine repetitive matrix protein 2",
  "gene_symbol": "SRRM2"
}